regulation of membrane permeability [GO:0090559] (biological process) Subtypes: regulation of mitochondrial membrane permeability [GO:0046902], regulation of lysosomal membrane permeability [GO:0097213], negative regulation of membrane permeability [GO:1905709], positive regulation of membrane permeability [GO:1905710] Definition: Any process that modulates the frequency, rate or extent of the passage or uptake of molecules by a membrane. References: PMID:22677064 Sources: GOC:kmv Relationships: is a type of regulation of biological quality [GO:0065008]